mannosylglycerate biosynthetic process [GO:0051479] (biological process) Sources: GOC:ai Definition: The chemical reactions and pathways resulting in the formation of mannosylglycerate, a very common compatible solute in thermophilic and hyperthermophilic organisms. Also known as: mannosylglycerate anabolism, mannosylglycerate biosynthesis, mannosylglycerate formation, mannosylglycerate synthesis Relationships: is a type of carbohydrate biosynthetic process [GO:0016051]; is a type of glycoside biosynthetic process [GO:0016138]; is a type of carboxylic acid biosynthetic process [GO:0046394]; is a type of mannosylglycerate metabolic process [GO:0051478]